{
  "gene_symbol": "OR51E2",
  "term_label": "Unknown biological process",
  "gene": "UniProtKB:Q9H255",
  "gene_name": "Olfactory receptor 51E2",
  "term_id": "UNKNOWN:0002"
}